carbamoyl-serine ammonia-lyase activity [GO:0047766] (molecular function) Also known as: O-carbamoyl-L-serine ammonia-lyase (decarboxylating; pyruvate-forming), O-carbamoyl-L-serine ammonia-lyase (pyruvate-forming), O-carbamoyl-L-serine deaminase activity, carbamoylserine deaminase activity Definition: Catalysis of the reaction: O-carbamoyl-L-serine + H2O + H+ = CO2 + 2 NH4 + pyruvate. Relationships: is a type of ammonia-lyase activity [GO:0016841] Sources: EC:4.3.1.13, RHEA:15445